spindle localization [GO:0051653] (biological process) Relationships: is a type of GO:0022402; is a type of organelle localization [GO:0051640] Definition: Any process in which is the spindle is transported to, and/or maintained in, a specific location. Subtypes: establishment of spindle localization [GO:0051293], maintenance of spindle location [GO:0051687] Sources: GOC:ai Also known as: establishment and maintenance of spindle localization, spindle localisation